detection of salicylic acid stimulus [GO:0009752] (biological process) Relationships: is a type of detection of chemical stimulus [GO:0009593]; is a type of response to salicylic acid [GO:0009751] Also known as: perception of salicylic acid stimulus Definition: The series of events in which a salicylic acid stimulus is received by a cell and converted into a molecular signal. Sources: GOC:sm